{
  "gene_symbol": "DGKG",
  "term_id": "GO:0005886",
  "gene": "UniProtKB:P49619",
  "gene_name": "Diacylglycerol kinase gamma",
  "term_label": "plasma membrane"
}